{
  "term_id": "GO:0000981",
  "gene_name": "Forkhead box protein L2",
  "gene_symbol": "FOXL2",
  "gene": "UniProtKB:P58012",
  "term_label": "DNA-binding transcription factor activity, RNA polymerase II-specific"
}